{
  "term_id": "GO:0005615",
  "gene_symbol": "PRTN3",
  "gene_name": "Myeloblastin",
  "term_label": "extracellular space",
  "gene": "UniProtKB:P24158"
}